{
  "gene_name": "Stathmin domain-containing protein 1",
  "gene_symbol": "STMND1",
  "term_label": "neuron projection",
  "gene": "UniProtKB:H3BQB6",
  "term_id": "GO:0043005"
}